{
  "gene_name": "Probable glutamate--tRNA ligase, mitochondrial",
  "gene": "UniProtKB:Q5JPH6",
  "gene_symbol": "EARS2",
  "term_id": "GO:0006424",
  "term_label": "glutamyl-tRNA aminoacylation"
}